{
  "term_id": "GO:0005886",
  "gene_symbol": "MYO1A",
  "term_label": "plasma membrane",
  "gene_name": "Unconventional myosin-Ia",
  "gene": "UniProtKB:Q9UBC5"
}